{
  "gene": "UniProtKB:Q9H2X0",
  "term_label": "negative regulation of BMP signaling pathway",
  "gene_name": "Chordin",
  "gene_symbol": "CHRD",
  "term_id": "GO:0030514"
}